{
  "gene_symbol": "SSTR1",
  "term_id": "GO:0071392",
  "term_label": "cellular response to estradiol stimulus",
  "gene": "UniProtKB:P30872",
  "gene_name": "Somatostatin receptor type 1"
}